fluconazole:proton antiporter activity [GO:0015313] (molecular function) Relationships: is a type of fluconazole transmembrane transporter activity [GO:0015244]; is a type of azole:proton antiporter activity [GO:0045119] Sources: TC:2.A.1.2.17 Also known as: fluconazole:hydrogen antiporter activity Definition: Enables the transfer of a solute or solutes from one side of a membrane to the other according to the reaction: H+(out) + fluconazole(in) = H+(in) + fluconazole(out).